{
  "term_label": "Unknown cellular component",
  "gene": "UniProtKB:Q9H1C7",
  "gene_symbol": "CYSTM1",
  "gene_name": "Cysteine-rich and transmembrane domain-containing protein 1",
  "term_id": "UNKNOWN:0003"
}